{
  "gene_name": "Vesicle transport protein SFT2C",
  "term_label": "Unknown cellular component",
  "gene_symbol": "SFT2D3",
  "gene": "UniProtKB:Q587I9",
  "term_id": "UNKNOWN:0003"
}